{
  "term_id": "UNKNOWN:0003",
  "gene_name": "Glucoside xylosyltransferase 2",
  "term_label": "Unknown cellular component",
  "gene_symbol": "GXYLT2",
  "gene": "UniProtKB:A0PJZ3"
}